EGFR-Grb2-Sos complex [GO:0070620] (cellular component) Relationships: is_a plasma membrane protein complex [GO:0098797] References: PMID:7798267, PMID:8940013 Sources: GOC:mah Definition: A protein complex that contains the epidermal growth factor receptor (EGFR), Grb2 and the guanine nucleotide exchange factor Sos (or an ortholog thereof, such as mSos1), and is involved in linking EGFR activation to the p21-Ras pathway. Also known as: Egfr-Grb2-mSos1 complex, EGF stimulated